{
  "gene_symbol": "PPP1R1A",
  "gene_name": "Protein phosphatase 1 regulatory subunit 1A",
  "term_label": "cytoplasm",
  "term_id": "GO:0005737",
  "gene": "UniProtKB:Q13522"
}